{
  "term_label": "negative regulation of single stranded viral RNA replication via double stranded DNA intermediate",
  "gene": "UniProtKB:Q6NTF7",
  "term_id": "GO:0045869",
  "gene_name": "DNA dC-dU-editing enzyme APOBEC-3H",
  "gene_symbol": "APOBEC3H"
}